{
  "gene": "UniProtKB:Q86VY4",
  "term_label": "chromatin",
  "gene_symbol": "TSPYL5",
  "gene_name": "Testis-specific Y-encoded-like protein 5",
  "term_id": "GO:0000785"
}